{
  "term_label": "Unknown biological process",
  "term_id": "UNKNOWN:0002",
  "gene_name": "Transmembrane protein 179",
  "gene": "UniProtKB:Q6ZVK1",
  "gene_symbol": "TMEM179"
}